{
  "gene_symbol": "ZNF254",
  "term_id": "GO:0000981",
  "gene_name": "Zinc finger protein 254",
  "gene": "UniProtKB:O75437",
  "term_label": "DNA-binding transcription factor activity, RNA polymerase II-specific"
}